{
  "gene_name": "Homeobox protein DBX1",
  "term_label": "cell differentiation in spinal cord",
  "gene_symbol": "DBX1",
  "gene": "UniProtKB:A6NMT0",
  "term_id": "GO:0021515"
}